{
  "term_label": "mRNA binding",
  "term_id": "GO:0003729",
  "gene": "UniProtKB:O94913",
  "gene_symbol": "PCF11",
  "gene_name": "Pre-mRNA cleavage complex 2 protein Pcf11"
}